{
  "gene_symbol": "TTI2",
  "gene": "UniProtKB:Q6NXR4",
  "term_id": "GO:0110078",
  "term_label": "TTT Hsp90 cochaperone complex",
  "gene_name": "TELO2-interacting protein 2"
}